regulation of delayed rectifier potassium channel activity [GO:1902259] (BP) Relationships: is a type of regulation of transmembrane transporter activity [GO:0022898]; regulates GO:0005251 Subtypes: negative regulation of delayed rectifier potassium channel activity [GO:1902260] References: PMID:11299204 Sources: GOC:BHF, GOC:TermGenie, GOC:rl Definition: Any process that modulates the frequency, rate or extent of delayed rectifier potassium channel activity.